{
  "gene_name": "Zinc transporter 6",
  "gene_symbol": "SLC30A6",
  "term_id": "GO:0005794",
  "term_label": "Golgi apparatus",
  "gene": "UniProtKB:Q6NXT4"
}